{
  "gene_name": "Bcl-2-modifying factor",
  "term_id": "GO:0010507",
  "gene": "UniProtKB:Q96LC9",
  "term_label": "negative regulation of autophagy",
  "gene_symbol": "BMF"
}